{
  "term_label": "Unknown cellular component",
  "gene_symbol": "FAM86C1P",
  "gene_name": "Putative protein FAM86C1P",
  "term_id": "UNKNOWN:0003",
  "gene": "UniProtKB:Q9NVL1"
}